{
  "gene_symbol": "SLC6A7",
  "gene": "UniProtKB:Q99884",
  "term_id": "GO:0005298",
  "gene_name": "Sodium-dependent proline transporter",
  "term_label": "proline:sodium symporter activity"
}